proximal/distal pattern formation involved in mesonephric nephron development [GO:0061226] (biological process) Relationships: is a type of GO:0061227; is a type of GO:0072047; is part of mesonephric nephron development [GO:0061215] Sources: GOC:mtg_kidney_jan10 Definition: The regionalization process in which specific areas of cell differentiation are determined along a proximal/distal axis of a nephron in the mesonephros. The proximal/distal axis is defined by a line that runs from the glomerulus (proximal end) outward toward the mesonephric duct (distal end).